{
  "gene_symbol": "Q6ZSN1",
  "term_label": "Unknown cellular component",
  "gene": "UniProtKB:Q6ZSN1",
  "term_id": "UNKNOWN:0003",
  "gene_name": "Putative uncharacterized protein FLJ45355"
}